T cell antigen processing and presentation [GO:0002457] (biological process) Definition: The process in which a T cell expresses antigen (peptide or lipid) on its cell surface in association with an MHC protein complex. Relationships: is a type of GO:0019882; is part of GO:0002456 Also known as: T lymphocyte antigen processing and presentation, T-cell antigen processing and presentation, T-lymphocyte antigen processing and presentation References: PMID:11417857, PMID:15120183 Sources: GOC:add Regulation: regulated by GO:0002625; negatively regulated by GO:0002626; positively regulated by positive regulation of T cell antigen processing and presentation [GO:0002627]